nuclear membrane disassembly [GO:0051081] (biological process) Subtypes: GO:0007077, sperm nuclear envelope removal [GO:0035040], meiotic nuclear membrane disassembly [GO:0051078] Also known as: nuclear envelope breakdown, nuclear envelope catabolism, nuclear envelope degradation, nuclear envelope disassembly Sources: GOC:ai Relationships: is a type of membrane disassembly [GO:0030397]; is a type of nuclear membrane organization [GO:0071763] Definition: The controlled breakdown of the nuclear membranes, for example during cellular division.